{
  "gene": "UniProtKB:Q9BTT4",
  "gene_name": "Mediator of RNA polymerase II transcription subunit 10",
  "gene_symbol": "MED10",
  "term_id": "UNKNOWN:0002",
  "term_label": "Unknown biological process"
}